oxidoreductase activity, acting on X-H and Y-H to form an X-Y bond, with oxygen as acceptor [GO:0046993] (molecular function) Definition: Catalysis of an oxidation-reduction (redox) reaction in which X-H and Y-H form X-Y and the acceptor is oxygen. Relationships: is a type of GO:0046992 Subtypes: isopenicillin-N synthase activity [GO:0016216], aureusidin synthase activity [GO:0033793], sulochrin oxidase [(+)-bisdechlorogeodin-forming] activity [GO:0047064], sulochrin oxidase [(-)-bisdechlorogeodin-forming] activity [GO:0047065], columbamine oxidase activity [GO:0050455], reticuline oxidase activity [GO:0050468], GO:0061686, GO:0102778, cannabidiolate synthase activity [GO:0102779] Sources: GOC:ai